{
  "term_label": "transcription repressor complex",
  "gene_symbol": "GMNN",
  "gene_name": "Geminin",
  "term_id": "GO:0017053",
  "gene": "UniProtKB:O75496"
}